{
  "gene_name": "Zinc finger protein 182",
  "gene_symbol": "ZNF182",
  "gene": "UniProtKB:P17025",
  "term_label": "RNA polymerase II cis-regulatory region sequence-specific DNA binding",
  "term_id": "GO:0000978"
}